pyroptosome complex [GO:0061703] (cellular component) Also known as: ASC pyroptosome Relationships: is a type of protein-containing complex [GO:0032991] References: PMID:17599095 Sources: GOC:dph Definition: A protein complex that consists of an assemble of ASC dimers that is capable of inducing pyroptosis.